{
  "gene": "UniProtKB:P15502",
  "term_label": "Unknown cellular component",
  "term_id": "UNKNOWN:0003",
  "gene_symbol": "ELN",
  "gene_name": "Elastin"
}